regulation of amide catabolic process [GO:0034251] (biological process) Also known as: regulation of amide breakdown, regulation of amide catabolism, regulation of amide degradation, regulation of cellular amide catabolic process Relationships: is a type of regulation of catabolic process [GO:0009894]; is a type of regulation of amide metabolic process [GO:0034248]; regulates GO:0043605 Sources: GOC:mah Subtypes: negative regulation of amide catabolic process [GO:0034252], GO:0034253, GO:0034254 Definition: Any process that modulates the frequency, rate or extent of the chemical reactions and pathways resulting in the breakdown of amides.